{
  "gene_name": "Tight junction protein ZO-2",
  "term_id": "GO:0090557",
  "term_label": "establishment of endothelial intestinal barrier",
  "gene": "UniProtKB:Q9UDY2",
  "gene_symbol": "TJP2"
}